symbiont-mediated suppression of host phagosome maturation [GO:0141158] (biological process) Definition: A process in which a symbiont inhibits or disrupts the normal maturation of host phagosomes. The host is defined as the larger of the organisms involved in a symbiotic interaction. References: PMID:21501366, PMID:30181274, PMID:30733336, PMID:30937925 Relationships: is a type of symbiont-mediated perturbation of host cellular process [GO:0044068]